{
  "gene_symbol": "SLA",
  "term_label": "phosphotyrosine residue binding",
  "gene": "UniProtKB:Q13239",
  "gene_name": "Src-like-adapter",
  "term_id": "GO:0001784"
}